{
  "term_id": "GO:0008017",
  "term_label": "microtubule binding",
  "gene_symbol": "REEP1",
  "gene_name": "Receptor expression-enhancing protein 1",
  "gene": "UniProtKB:Q9H902"
}